{
  "gene_name": "Neuromodulin",
  "term_label": "cytoplasm",
  "term_id": "GO:0005737",
  "gene_symbol": "GAP43",
  "gene": "UniProtKB:P17677"
}